{
  "gene_name": "Nuclear receptor-binding protein",
  "gene": "UniProtKB:Q9UHY1",
  "gene_symbol": "NRBP1",
  "term_id": "GO:1904062",
  "term_label": "regulation of monoatomic cation transmembrane transport"
}